{
  "term_id": "GO:0005634",
  "term_label": "nucleus",
  "gene_symbol": "ATF7IP2",
  "gene_name": "Activating transcription factor 7-interacting protein 2",
  "gene": "UniProtKB:Q5U623"
}